{
  "gene_symbol": "SSX7",
  "term_id": "UNKNOWN:0001",
  "gene": "UniProtKB:Q7RTT5",
  "term_label": "Unknown molecular function",
  "gene_name": "Protein SSX7"
}